{
  "term_label": "single-stranded DNA binding",
  "term_id": "GO:0003697",
  "gene": "UniProtKB:Q53H47",
  "gene_symbol": "SETMAR",
  "gene_name": "Histone-lysine N-methyltransferase SETMAR"
}